cellular response to trehalose-6-phosphate stimulus [GO:0071330] (biological process) Relationships: is a type of GO:0071324; is a type of response to trehalose-6-phosphate [GO:0080094] Sources: GOC:mah Definition: Any process that results in a change in state or activity of a cell (in terms of movement, secretion, enzyme production, gene expression, etc.) as a result of a trehalose-6-phosphate stimulus.